{
  "gene": "UniProtKB:Q5TC82",
  "term_label": "mRNA binding",
  "gene_symbol": "RC3H1",
  "gene_name": "Roquin-1",
  "term_id": "GO:0003729"
}